3-aminobutyryl-CoA ammonia-lyase activity [GO:0047459] (molecular function) Definition: Catalysis of the reaction: (S)-3-aminobutanoyl-CoA = crotonoyl-CoA + NH4. Relationships: is a type of ammonia-lyase activity [GO:0016841] Sources: EC:4.3.1.14, RHEA:10056 Also known as: L-3-aminobutyryl-CoA ammonia-lyase (crotonoyl-CoA-forming), L-3-aminobutyryl-CoA ammonia-lyase activity, L-3-aminobutyryl-CoA deaminase activity